{
  "gene_name": "Acylglycerol kinase, mitochondrial",
  "term_id": "GO:0047620",
  "gene": "UniProtKB:Q53H12",
  "term_label": "acylglycerol kinase activity",
  "gene_symbol": "AGK"
}